{
  "gene": "UniProtKB:Q92552",
  "gene_symbol": "MRPS27",
  "gene_name": "Small ribosomal subunit protein mS27",
  "term_id": "GO:0005739",
  "term_label": "mitochondrion"
}